sequence-specific DNA binding, bending [GO:0044374] (molecular function) Sources: GOC:jl, GOC:vw Relationships: is_a GO:0008301; is a type of sequence-specific double-stranded DNA binding [GO:1990837] Subtypes: RNA polymerase II cis-regulatory region sequence-specific DNA binding, bending [GO:0044377], rDNA spacer replication fork barrier binding, bending [GO:0110035] Definition: The activity of binding selectively and non-covalently to DNA in a sequence-specific manner and distorting the original structure of DNA, typically a straight helix, into a bend, or increasing the bend if the original structure was intrinsically bent due to its sequence. Also known as: DNA bending involving sequence-specific DNA binding